glucosinolate biosynthetic process from homomethionine [GO:0033506] (biological process) Relationships: is a type of carboxylic acid metabolic process [GO:0019752]; is a type of GO:0019761 Sources: GOC:mah, MetaCyc:PWY-1187 Also known as: glucosinolate anabolism from homomethionine, glucosinolate biosynthesis from homomethionine, glucosinolate formation from homomethionine, glucosinolate synthesis from homomethionine Definition: The chemical reactions and pathways resulting in the formation of glucosinolates from other compounds including homomethionine.